{
  "gene": "UniProtKB:P02144",
  "gene_name": "Myoglobin",
  "term_label": "skeletal muscle contraction",
  "gene_symbol": "MB",
  "term_id": "GO:0003009"
}